{
  "gene_name": "Alpha-1A adrenergic receptor",
  "term_id": "GO:0007200",
  "gene": "UniProtKB:P35348",
  "term_label": "phospholipase C-activating G protein-coupled receptor signaling pathway",
  "gene_symbol": "ADRA1A"
}